{
  "gene_symbol": "DHRS13",
  "gene_name": "Dehydrogenase_reductase SDR family member 13",
  "term_label": "Unknown cellular component",
  "term_id": "UNKNOWN:0003",
  "gene": "UniProtKB:Q6UX07"
}